{
  "term_id": "GO:0045332",
  "gene": "UniProtKB:P21439",
  "gene_name": "Phosphatidylcholine translocator ABCB4",
  "term_label": "phospholipid translocation",
  "gene_symbol": "ABCB4"
}